{
  "gene": "UniProtKB:Q8IY22",
  "term_label": "Unknown molecular function",
  "gene_name": "C-Maf-inducing protein",
  "gene_symbol": "CMIP",
  "term_id": "UNKNOWN:0001"
}